{
  "gene_symbol": "CYP11B1",
  "term_label": "corticosterone 18-monooxygenase activity",
  "term_id": "GO:0047783",
  "gene_name": "Cytochrome P450 11B1, mitochondrial",
  "gene": "UniProtKB:P15538"
}